{
  "gene_name": "B-cell receptor CD22",
  "term_id": "GO:0042113",
  "gene_symbol": "CD22",
  "term_label": "B cell activation",
  "gene": "UniProtKB:P20273"
}